negative regulation of immune effector process [GO:0002698] (biological process) Sources: GOC:add Also known as: down regulation of immune effector process, down-regulation of immune effector process, downregulation of immune effector process, inhibition of immune effector process Definition: Any process that stops, prevents, or reduces the frequency, rate, or extent of an immune effector process. Subtypes: negative regulation of granuloma formation [GO:0002632], GO:0002701, negative regulation of leukocyte mediated immunity [GO:0002704], GO:0032821, negative regulation of natural killer cell differentiation involved in immune response [GO:0032827], negative regulation of CD4-positive, CD25-positive, alpha-beta regulatory T cell differentiation involved in immune response [GO:0032833], negative regulation of mast cell activation involved in immune response [GO:0033007], negative regulation of leukocyte degranulation [GO:0043301], negative regulation of memory T cell differentiation [GO:0043381], negative regulation of T-helper cell differentiation [GO:0045623], negative regulation of complement activation [GO:0045916], negative regulation of respiratory burst involved in inflammatory response [GO:0060266], GO:0140540, GO:1900099, negative regulation of Fc-gamma receptor signaling pathway involved in phagocytosis [GO:1905450], negative regulation of T cell activation via T cell receptor contact with antigen bound to MHC molecule on antigen presenting cell [GO:2001189], negative regulation of gamma-delta T cell activation involved in immune response [GO:2001192] Relationships: is a type of negative regulation of immune system process [GO:0002683]; is a type of regulation of immune effector process [GO:0002697]; negatively regulates GO:0002252